{
  "gene_symbol": "TENT5B",
  "gene": "UniProtKB:Q96A09",
  "term_id": "GO:0048255",
  "gene_name": "Terminal nucleotidyltransferase 5B",
  "term_label": "mRNA stabilization"
}